mRNA modification [GO:0016556] (biological process) Note: The term 'RNA editing' (GO:0016547) was merged into 'RNA modification' (GO:0009451) on the basis of statements in the preface of Modification and Editing of RNA (ISBN:1555811337) that there is no clear distinction between modification and editing. Parallel changes were made for substrate (e.g. tRNA, rRNA, etc.) specific child terms of 'RNA editing'. Definition: The covalent alteration of one or more nucleotides within an mRNA molecule to produce an mRNA molecule with a sequence that differs from that coded genetically. Relationships: is a type of RNA modification [GO:0009451]; is a type of mRNA metabolic process [GO:0016071] Also known as: mRNA editing Subtypes: GO:0080156, chloroplast mRNA modification [GO:1900871], mRNA pseudouridine synthesis [GO:1990481] Sources: GOC:curators Regulation: regulated by regulation of mRNA modification [GO:0090365]; positively regulated by positive regulation of mRNA modification [GO:0090366]; negatively regulated by negative regulation of mRNA modification [GO:0090367]